{
  "gene": "UniProtKB:Q8NG41",
  "term_label": "Unknown cellular component",
  "gene_symbol": "NPB",
  "term_id": "UNKNOWN:0003",
  "gene_name": "Neuropeptide B"
}